amorpha-4,11-diene synthase activity [GO:0034006] (molecular function) Sources: EC:4.2.3.24, RHEA:18325 Relationships: is a type of sesquiterpene synthase activity [GO:0010334] Also known as: 2-trans,6-trans-farnesyl-diphosphate diphosphate-lyase (amorpha-4,11-diene-forming) activity, amorphadiene synthase activity Definition: Catalysis of the reaction: 2-trans,6-trans-farnesyl diphosphate = amorpha-4,11-diene + diphosphate.